{
  "gene_name": "Ropporin-1-like protein",
  "gene_symbol": "ROPN1L",
  "gene": "UniProtKB:Q96C74",
  "term_id": "GO:0005737",
  "term_label": "cytoplasm"
}